{
  "gene": "UniProtKB:Q9ULD2",
  "term_label": "microtubule binding",
  "gene_name": "Microtubule-associated tumor suppressor 1",
  "term_id": "GO:0008017",
  "gene_symbol": "MTUS1"
}